Golgi vesicle bud deformation and release [GO:0048198] (biological process) Definition: The process in which cytosolic coat proteins fit together in a basketlike convex framework to form a coated deformed region on the cytoplasmic surface of the membrane. The deformed region forms into a complete vesicle and is released. References: PMID:10219233 Sources: GOC:jid, ISBN:0716731363 Also known as: Golgi-derived vesicle bud deformation and release, dictyosome vesicle bud deformation Relationships: is a type of membrane organization [GO:0061024]; is part of Golgi vesicle budding [GO:0048194]